RNP body [GO:0140365] (cellular component) Also known as: BR-body Relationships: is a type of cytoplasmic ribonucleoprotein granule [GO:0036464] References: PMID:30197298 Definition: A ribonucleoprotein granule located in the cytoplasm of bacteria, minimally containing the RNase E protein and RNA molecules. Bacterial RNP-bodies are similar to eukaryotic P-bodies and stress granules.